{
  "term_id": "UNKNOWN:0002",
  "gene": "UniProtKB:A6NKN8",
  "gene_symbol": "PCP4L1",
  "term_label": "Unknown biological process",
  "gene_name": "Purkinje cell protein 4-like protein 1"
}